{
  "term_label": "olfactory receptor activity",
  "gene_name": "Olfactory receptor 52M1",
  "gene": "UniProtKB:Q8NGK5",
  "term_id": "GO:0004984",
  "gene_symbol": "OR52M1"
}